{
  "gene_symbol": "GID8",
  "term_label": "nucleus",
  "gene_name": "Glucose-induced degradation protein 8 homolog",
  "gene": "UniProtKB:Q9NWU2",
  "term_id": "GO:0005634"
}